{
  "gene": "UniProtKB:Q6V0I7",
  "gene_name": "Protocadherin Fat 4",
  "gene_symbol": "FAT4",
  "term_label": "epithelial cell differentiation",
  "term_id": "GO:0030855"
}